{
  "term_id": "GO:0005886",
  "term_label": "plasma membrane",
  "gene": "UniProtKB:Q96KG7",
  "gene_name": "Multiple epidermal growth factor-like domains protein 10",
  "gene_symbol": "MEGF10"
}